{
  "term_label": "cilium assembly",
  "term_id": "GO:0060271",
  "gene": "UniProtKB:Q96GX1",
  "gene_symbol": "TCTN2",
  "gene_name": "Tectonic-2"
}